{
  "gene_symbol": "SLC9B1",
  "gene": "UniProtKB:Q4ZJI4",
  "term_label": "Unknown molecular function",
  "gene_name": "Sodium_hydrogen exchanger 9B1",
  "term_id": "UNKNOWN:0001"
}